{
  "term_label": "Unknown biological process",
  "gene_symbol": "LRRTM2",
  "term_id": "UNKNOWN:0002",
  "gene": "UniProtKB:O43300",
  "gene_name": "Leucine-rich repeat transmembrane neuronal protein 2"
}